{
  "term_id": "GO:0061630",
  "term_label": "ubiquitin protein ligase activity",
  "gene": "UniProtKB:Q9NS56",
  "gene_symbol": "TOPORS",
  "gene_name": "E3 ubiquitin-protein ligase Topors"
}